sensory perception of low humidity [GO:0098511] (biological process) References: PMID:18269908 Definition: The series of events required for an organism to detect low environmental humidity, convert this detection into a molecular signal, and recognize and characterize the signal. This is a neurological process. Relationships: is a type of sensory perception of humidity [GO:0098509]